foraging behavior by probing substrate [GO:0060758] (biological process) Sources: GOC:dph, GOC:tb Relationships: is a type of foraging behavior [GO:0060756] Definition: Foraging behavior in which an anatomical part of the organism is inserted into the substrate to locate food.